{
  "gene_symbol": "GLI3",
  "term_label": "regulation of transcription by RNA polymerase II",
  "gene_name": "Transcriptional activator GLI3",
  "gene": "UniProtKB:P10071",
  "term_id": "GO:0006357"
}